response to metformin [GO:1901558] (biological process) Relationships: is a type of response to nitrogen compound [GO:1901698] Definition: Any process that results in a change in state or activity of a cell or an organism (in terms of movement, secretion, enzyme production, gene expression, etc.) as a result of a metformin stimulus. Sources: GOC:TermGenie